negative regulation of type IIa hypersensitivity [GO:0001797] (biological process) Sources: GOC:add, ISBN:0781735149 Relationships: is a type of regulation of type IIa hypersensitivity [GO:0001796]; is a type of negative regulation of type II hypersensitivity [GO:0002893]; negatively regulates GO:0001794 Also known as: down regulation of type IIa hypersensitivity, down-regulation of type IIa hypersensitivity, downregulation of type IIa hypersensitivity, inhibition of type IIa hypersensitivity Definition: Any process that stops, prevents, or reduces the rate of type IIa hypersensitivity, a type of inflammatory response. Subtypes: negative regulation of antibody-dependent cellular cytotoxicity [GO:0001814]